{
  "term_label": "phagophore assembly site",
  "gene_name": "Serine_threonine-protein kinase ULK1",
  "gene": "UniProtKB:O75385",
  "term_id": "GO:0000407",
  "gene_symbol": "ULK1"
}